{
  "term_id": "UNKNOWN:0002",
  "gene": "UniProtKB:P0DV79",
  "term_label": "Unknown biological process",
  "gene_name": "Speedy protein E18",
  "gene_symbol": "SPDYE18"
}